pointed-end actin filament capping [GO:0051694] (biological process) Also known as: minus-end F-actin capping activity, minus-end actin filament capping activity, pointed-end F-actin capping activity, pointed-end actin capping activity Relationships: is a type of actin filament capping [GO:0051693] Definition: The binding of a protein or protein complex to the pointed (or minus) end of an actin filament, thus preventing the addition, exchange or removal of further actin subunits. Sources: ISBN:071673706X